positive regulation of SMAD protein signal transduction [GO:0060391] (biological process) Sources: GOC:BHF, GOC:dph, GOC:tb Also known as: positive regulation of SMAD protein import into nucleus, positive regulation of SMAD protein nuclear translocation Relationships: is a type of regulation of SMAD protein signal transduction [GO:0060390]; is a type of positive regulation of transmembrane receptor protein serine/threonine kinase signaling pathway [GO:0090100]; is a type of positive regulation of intracellular signal transduction [GO:1902533]; positively regulates SMAD protein signal transduction [GO:0060395] Definition: Any process that increases the rate, frequency or extent of SMAD protein signal transduction.